{
  "gene_name": "Metal cation symporter ZIP14",
  "gene": "UniProtKB:Q15043",
  "term_label": "intracellular monoatomic cation homeostasis",
  "term_id": "GO:0030003",
  "gene_symbol": "SLC39A14"
}